{
  "term_id": "GO:0048167",
  "gene_symbol": "RASGRF1",
  "gene_name": "Ras-specific guanine nucleotide-releasing factor 1",
  "term_label": "regulation of synaptic plasticity",
  "gene": "UniProtKB:Q13972"
}